{
  "gene_name": "Vomeronasal type-1 receptor 5",
  "term_id": "GO:0005550",
  "gene_symbol": "VN1R5",
  "term_label": "pheromone binding",
  "gene": "UniProtKB:Q7Z5H4"
}